{
  "gene": "UniProtKB:O95257",
  "term_label": "nucleus",
  "gene_symbol": "GADD45G",
  "gene_name": "Growth arrest and DNA damage-inducible protein GADD45 gamma",
  "term_id": "GO:0005634"
}